{
  "term_label": "U4 snRNA binding",
  "gene_symbol": "PRPF4",
  "term_id": "GO:0030621",
  "gene_name": "U4_U6 small nuclear ribonucleoprotein Prp4",
  "gene": "UniProtKB:O43172"
}